isoleucine transmembrane transport [GO:1903714] (biological process) Relationships: is a type of GO:0003333; is a type of isoleucine transport [GO:0015818]; is a type of carboxylic acid transmembrane transport [GO:1905039] References: PMID:18503766 Sources: GOC:TermGenie, GO_REF:0000069 Definition: The directed movement of isoleucine across a membrane by means of some agent such as a transporter or a pore. Subtypes: L-isoleucine import across plasma membrane [GO:1903806]